{
  "gene": "UniProtKB:A7E2F4",
  "gene_symbol": "GOLGA8A",
  "term_id": "GO:0005801",
  "term_label": "cis-Golgi network",
  "gene_name": "Golgin subfamily A member 8A"
}